VCP-NSFL1C complex [GO:1990730] (cellular component) Definition: A protein complex between the ATPase VCP (p97) and its cofactor p47 (NSFL1C). In human, the protein complex consists of one homotrimer of NSFL1C/p47 per homohexamer of VCP/p97. References: PMID:9214505 Sources: GOC:PARL, GOC:bf Also known as: p97-p47 complex Relationships: is_a protein-containing complex [GO:0032991]; BFO_0000050 cytoplasm [GO:0005737]